{
  "term_label": "RNA polymerase II cis-regulatory region sequence-specific DNA binding",
  "gene": "UniProtKB:P56693",
  "gene_name": "Transcription factor SOX-10",
  "gene_symbol": "SOX10",
  "term_id": "GO:0000978"
}